{
  "term_id": "GO:0017005",
  "term_label": "3'-tyrosyl-DNA phosphodiesterase activity",
  "gene_symbol": "TDP1",
  "gene": "UniProtKB:Q9NUW8",
  "gene_name": "Tyrosyl-DNA phosphodiesterase 1"
}